{
  "gene": "UniProtKB:Q5J5C9",
  "term_label": "membrane destabilizing activity",
  "gene_symbol": "DEFB121",
  "term_id": "GO:0140912",
  "gene_name": "Beta-defensin 121"
}